{
  "gene": "UniProtKB:Q969V5",
  "gene_symbol": "MUL1",
  "term_id": "GO:0090141",
  "term_label": "positive regulation of mitochondrial fission",
  "gene_name": "Mitochondrial ubiquitin ligase activator of NFKB 1"
}